{
  "gene_name": "Cochlin",
  "gene": "UniProtKB:O43405",
  "gene_symbol": "COCH",
  "term_id": "GO:0031012",
  "term_label": "extracellular matrix"
}